{
  "term_label": "nucleus",
  "gene_symbol": "ZNF426",
  "term_id": "GO:0005634",
  "gene": "UniProtKB:Q9BUY5",
  "gene_name": "Zinc finger protein 426"
}